{
  "gene_symbol": "ZNF517",
  "term_id": "GO:0000981",
  "term_label": "DNA-binding transcription factor activity, RNA polymerase II-specific",
  "gene": "UniProtKB:Q6ZMY9",
  "gene_name": "Zinc finger protein 517"
}